{
  "term_id": "GO:0051453",
  "term_label": "regulation of intracellular pH",
  "gene_name": "Sodium_hydrogen exchanger 6",
  "gene": "UniProtKB:Q92581",
  "gene_symbol": "SLC9A6"
}